{
  "gene_symbol": "AGFG2",
  "term_id": "GO:0001675",
  "term_label": "acrosome assembly",
  "gene": "UniProtKB:O95081",
  "gene_name": "Arf-GAP domain and FG repeat-containing protein 2"
}